{
  "gene_symbol": "MYEF2",
  "gene_name": "Myelin expression factor 2",
  "term_label": "nucleus",
  "term_id": "GO:0005634",
  "gene": "UniProtKB:Q9P2K5"
}